{
  "term_id": "UNKNOWN:0002",
  "gene_symbol": "Q6P435",
  "gene_name": "Putative uncharacterized SMG1-like protein",
  "term_label": "Unknown biological process",
  "gene": "UniProtKB:Q6P435"
}